neuroblast migration [GO:0097402] (biological process) References: PMID:15543145 Sources: CL:0000031, GOC:jc Regulation: regulated by GO:0061853; positively regulated by positive regulation of neuroblast migration [GO:0061854]; negatively regulated by negative regulation of neuroblast migration [GO:0061855] Relationships: is a type of cell migration [GO:0016477] Definition: The orderly movement of a neuroblast from one site to another, often during the development of a multicellular organism or multicellular structure. A neuroblast is any cell that will divide and give rise to a neuron.